response to bacterium [GO:0009617] (biological process) Definition: Any process that results in a change in state or activity of a cell or an organism (in terms of movement, secretion, enzyme production, gene expression, etc.) as a result of a stimulus from a bacterium. Relationships: is a type of response to other organism [GO:0051707] Subtypes: response to symbiotic bacterium [GO:0009609], detection of bacterium [GO:0016045], GO:0042742, response to Gram-positive bacterium [GO:0140459], response to Gram-negative bacterium [GO:0140460] Sources: GOC:hb Also known as: response to bacteria